{
  "term_id": "GO:0008017",
  "term_label": "microtubule binding",
  "gene": "UniProtKB:Q8N5G2",
  "gene_name": "Macoilin",
  "gene_symbol": "MACO1"
}